{
  "gene": "UniProtKB:Q9P2X3",
  "term_label": "Unknown molecular function",
  "gene_symbol": "IMPACT",
  "term_id": "UNKNOWN:0001",
  "gene_name": "Protein IMPACT"
}